antigen sampling in mucosal-associated lymphoid tissue [GO:0002404] (biological process) Definition: The process of apical-to-basolateral delivery of soluble and particulate antigens to underlying mucosal-associated lymphoid tissue. Also known as: antigen sampling in MALT, antigen transport in MALT, antigen transport in mucosal-associated lymphoid tissue References: PMID:11896763, PMID:12843411, PMID:15681746 Sources: GOC:jal Relationships: is a type of immune system process [GO:0002376]; is part of mucosal immune response [GO:0002385] Subtypes: antigen sampling by dendritic cells in mucosal-associated lymphoid tissue [GO:0002405], antigen sampling by M cells in mucosal-associated lymphoid tissue [GO:0002406]